zinc ion transmembrane transport [GO:0071577] (biological process) Definition: A process in which a zinc II ion is transported from one side of a membrane to the other by means of some agent such as a transporter or pore. Sources: GOC:BHF, GOC:mah Also known as: zinc II ion transmembrane transport, zinc ion membrane transport, zinc transmembrane transport Note: Note that this term is not intended for use in annotating lateral movement within membranes. Relationships: is a type of GO:0006829; is a type of monoatomic cation transmembrane transport [GO:0098655] Subtypes: zinc ion import into organelle [GO:0062111], zinc ion import across plasma membrane [GO:0071578], zinc ion export from vacuole [GO:0140147], zinc export across plasma membrane [GO:0140882] Regulation: regulated by regulation of zinc ion transmembrane transport [GO:0071580]; negatively regulated by negative regulation of zinc ion transmembrane transport [GO:0071583]